creatininase activity [GO:0047789] (molecular function) Definition: Catalysis of the reaction: creatinine + H2O = creatine. Sources: EC:3.5.2.10, RHEA:14533 Also known as: creatinine hydrolase, creatinine amidohydrolase activity Relationships: is a type of hydrolase activity, acting on carbon-nitrogen (but not peptide) bonds, in cyclic amides [GO:0016812]